response to sterol [GO:0036314] (biological process) Relationships: is a type of response to lipid [GO:0033993]; is a type of response to oxygen-containing compound [GO:1901700] Definition: Any process that results in a change in state or activity of a cell or an organism (in terms of movement, secretion, enzyme production, gene expression, etc.) as a result of a sterol stimulus. Sources: GOC:bf Subtypes: response to ecdysone [GO:0035075], cellular response to sterol [GO:0036315], GO:0070723, GO:1905092